{
  "gene_symbol": "CEP95",
  "term_label": "Unknown molecular function",
  "gene_name": "Centrosomal protein of 95 kDa",
  "gene": "UniProtKB:Q96GE4",
  "term_id": "UNKNOWN:0001"
}